negative regulation of microvillus length [GO:1903982] (biological process) Also known as: down regulation of regulation of microvillus length, down-regulation of regulation of microvillus length, downregulation of regulation of microvillus length, inhibition of regulation of microvillus length Relationships: is a type of negative regulation of cell projection organization [GO:0031345]; is a type of regulation of microvillus length [GO:0032532] References: PMID:22114352 Sources: GOC:als Definition: A process that decreases the length of a microvillus.